{
  "gene_symbol": "SPDYE5",
  "gene": "UniProtKB:A6NIY4",
  "gene_name": "Speedy protein E5",
  "term_label": "Unknown cellular component",
  "term_id": "UNKNOWN:0003"
}